inositol bisphosphate phosphatase activity [GO:0016312] (molecular function) Definition: Catalysis of the reaction: myo-inositol bisphosphate + H2O = myo-inositol phosphate + phosphate. Sources: GOC:hb Relationships: is a type of GO:0052745 Subtypes: inositol-1,4-bisphosphate 1-phosphatase activity [GO:0004441], inositol-4,5-bisphosphate 5-phosphatase activity [GO:0030487], GO:0052828